{
  "gene": "UniProtKB:Q13093",
  "term_id": "UNKNOWN:0003",
  "gene_name": "Platelet-activating factor acetylhydrolase",
  "term_label": "Unknown cellular component",
  "gene_symbol": "PLA2G7"
}